regulation of plasmacytoid dendritic cell cytokine production [GO:0002736] (biological process) Subtypes: negative regulation of plasmacytoid dendritic cell cytokine production [GO:0002737], positive regulation of plasmacytoid dendritic cell cytokine production [GO:0002738] Relationships: is a type of GO:0002730; regulates plasmacytoid dendritic cell cytokine production [GO:0002373] Sources: GOC:add Definition: Any process that modulates the frequency, rate, or extent of plasmacytoid dendritic cell cytokine production.